RNA acetylation [GO:1990884] (BP) Relationships: is_a RNA modification [GO:0009451] Subtypes: tRNA acetylation [GO:0051391], rRNA acetylation [GO:1990882] Definition: The posttranscriptional addition of one or more acetyl groups to specific residues in an RNA molecule. References: PMID:25402480